{
  "gene": "UniProtKB:O15169",
  "gene_symbol": "AXIN1",
  "term_id": "GO:0008013",
  "gene_name": "Axin-1",
  "term_label": "beta-catenin binding"
}